{
  "gene": "UniProtKB:A0A075B7D8",
  "gene_name": "Immunoglobulin heavy variable 3_OR15-7 (pseudogene) (Fragment)",
  "gene_symbol": "IGHV3OR15-7",
  "term_id": "UNKNOWN:0003",
  "term_label": "Unknown cellular component"
}